{
  "gene_name": "Suppressor of cytokine signaling 2",
  "term_label": "cytokine-mediated signaling pathway",
  "term_id": "GO:0019221",
  "gene": "UniProtKB:O14508",
  "gene_symbol": "SOCS2"
}